positive regulation of lymphocyte proliferation [GO:0050671] (biological process) Sources: GOC:ai Also known as: up regulation of lymphocyte proliferation, up-regulation of lymphocyte proliferation, upregulation of lymphocyte proliferation, activation of lymphocyte proliferation, stimulation of lymphocyte proliferation Definition: Any process that activates or increases the rate or extent of lymphocyte proliferation. Relationships: is a type of positive regulation of mononuclear cell proliferation [GO:0032946]; is a type of regulation of lymphocyte proliferation [GO:0050670]; is_a positive regulation of lymphocyte activation [GO:0051251]; positively regulates GO:0046651 Subtypes: positive regulation of B cell proliferation [GO:0030890], positive regulation of natural killer cell proliferation [GO:0032819], positive regulation of T cell proliferation [GO:0042102]